isopiperitenol dehydrogenase activity [GO:0018458] (molecular function) Definition: Catalysis of the reaction: (1S,6R)-isopiperitenol + NAD+ = (6R)-isoperitenone + H+ + NADH. Also known as: (-)-trans-isopiperitenol:NAD+ oxidoreductase activity Sources: EC:1.1.1.223, RHEA:20860 Relationships: is a type of GO:0016616